{
  "gene": "UniProtKB:O75023",
  "term_id": "GO:0032396",
  "gene_symbol": "LILRB5",
  "term_label": "inhibitory MHC class I receptor activity",
  "gene_name": "Leukocyte immunoglobulin-like receptor subfamily B member 5"
}